regulation of spontaneous neurotransmitter secretion [GO:1904048] (biological process) References: PMID:22314364 Sources: GOC:PARL, GOC:TermGenie, GOC:pad, GO_REF:0000058 Subtypes: negative regulation of spontaneous neurotransmitter secretion [GO:1904049], positive regulation of spontaneous neurotransmitter secretion [GO:1904050] Note: An example of this is PARK2 / parkin in human (O60260) in PMID:22314364 (inferred from mutant phenotype). Also known as: regulation of stimulus-independent neurotransmitter secretion Definition: Any process that modulates the frequency, rate or extent of spontaneous neurotransmitter secretion. Relationships: is a type of regulation of neurotransmitter secretion [GO:0046928]; is a type of regulation of spontaneous synaptic transmission [GO:0150003]; regulates spontaneous neurotransmitter secretion [GO:0061669]